{
  "gene_symbol": "SLC6A11",
  "term_id": "GO:0006865",
  "gene": "UniProtKB:P48066",
  "term_label": "amino acid transport",
  "gene_name": "Sodium- and chloride-dependent GABA transporter 3"
}